sodium:galactoside symporter activity [GO:0044669] (molecular function) Relationships: is a type of solute:sodium symporter activity [GO:0015370]; is_a carbohydrate derivative transmembrane transporter activity [GO:1901505] Sources: GOC:crds Definition: Enables the transfer of a solute or solutes from one side of a membrane to the other according to the reaction: sodium(out)+ galactoside(out) = sodium(in) + galactoside(in).